{
  "term_id": "GO:0048731",
  "gene_name": "Developmental pluripotency-associated protein 4",
  "gene_symbol": "DPPA4",
  "gene": "UniProtKB:Q7L190",
  "term_label": "system development"
}